negative regulation of epinephrine uptake [GO:0051627] (biological process) Definition: Any process that stops, prevents, or reduces the frequency, rate or extent of the directed movement of epinephrine into a cell. Sources: GOC:ai Also known as: down regulation of epinephrine uptake, down-regulation of epinephrine uptake, downregulation of epinephrine uptake, negative regulation of adrenaline uptake, negative regulation of epinephrine import Relationships: is a type of GO:0051051; is a type of GO:0051626; negatively regulates epinephrine uptake [GO:0051625] Subtypes: GO:0051629